{
  "term_id": "GO:0021675",
  "gene": "UniProtKB:P01138",
  "gene_symbol": "NGF",
  "term_label": "nerve development",
  "gene_name": "Beta-nerve growth factor"
}